{
  "term_label": "Unknown molecular function",
  "term_id": "UNKNOWN:0001",
  "gene_name": "Proline-rich protein 7",
  "gene_symbol": "PRR7",
  "gene": "UniProtKB:Q8TB68"
}